{
  "term_id": "GO:0004128",
  "gene_name": "NADH-cytochrome b5 reductase 2",
  "gene": "UniProtKB:Q6BCY4",
  "gene_symbol": "CYB5R2",
  "term_label": "cytochrome-b5 reductase activity, acting on NAD(P)H"
}